decarboxylation-driven active transmembrane transporter activity [GO:0015451] (molecular function) Definition: Primary active transport of a solute across a membrane driven by decarboxylation of a cytoplasmic substrate. Primary active transport is catalysis of the transport of a solute across a membrane, up the solute's concentration gradient, by binding the solute and undergoing a series of conformational changes. Transport works equally well in either direction and is driven by a primary energy source. Sources: GOC:mtg_transport, ISBN:0815340729, TC:3.B.-.-.- Also known as: decarboxylation-driven transporter Relationships: is a type of primary active transmembrane transporter activity [GO:0015399]; has part GO:0016831 Subtypes: glutaconyl-CoA decarboxylase activity [GO:0018801]